Entner-Doudoroff pathway through gluconate [GO:0061679] (biological process) Definition: The Entner-Doudoroff pathway that proceeds through a D-gluconate intermediate. References: PMID:12921536 Sources: GOC:dph Also known as: gluconate pathway Relationships: is a type of Entner-Doudoroff pathway [GO:0061678]; has part gluconate dehydratase activity [GO:0047929]; BFO_0000051 glucose 1-dehydrogenase (NADP+) activity [GO:0047935] Subtypes: Entner-Doudoroff pathway through gluconate to D-glyceraldehyde [GO:0061680], Entner-Doudoroff pathway through gluconate to D-glyceraldehyde-3-phosphate [GO:0061681]